endocardial cell development [GO:0060958] (biological process) Definition: The progression of an endocardial cell over time, from its formation to the mature cell. An endocardial cell is a specialized endothelial cell that makes up the endocardium portion of the heart. Sources: GOC:mtg_heart Relationships: is a type of endothelial cell development [GO:0001885]; is_a cardiac cell development [GO:0055006]; is part of endocardial cell differentiation [GO:0060956]